{
  "term_label": "cytoplasm",
  "term_id": "GO:0005737",
  "gene": "UniProtKB:Q9P0V3",
  "gene_name": "SH3 domain-binding protein 4",
  "gene_symbol": "SH3BP4"
}